{
  "gene_symbol": "ZNF543",
  "gene": "UniProtKB:Q08ER8",
  "gene_name": "Zinc finger protein 543",
  "term_label": "nucleus",
  "term_id": "GO:0005634"
}